{
  "term_label": "organelle transport along microtubule",
  "gene_name": "Coatomer subunit gamma-2",
  "gene": "UniProtKB:Q9UBF2",
  "term_id": "GO:0072384",
  "gene_symbol": "COPG2"
}